{
  "gene_symbol": "TRIB3",
  "gene": "UniProtKB:Q96RU7",
  "term_id": "GO:0032436",
  "gene_name": "Tribbles homolog 3",
  "term_label": "positive regulation of proteasomal ubiquitin-dependent protein catabolic process"
}